{
  "term_label": "glutamate dehydrogenase (NAD+) activity",
  "gene_symbol": "GLUD1",
  "term_id": "GO:0004352",
  "gene_name": "Glutamate dehydrogenase 1, mitochondrial",
  "gene": "UniProtKB:P00367"
}